{
  "gene": "UniProtKB:Q99835",
  "term_id": "GO:0005113",
  "gene_name": "Protein smoothened",
  "gene_symbol": "SMO",
  "term_label": "patched binding"
}